nicotinamide-nucleotide adenylyltransferase activity [GO:0000309] (molecular function) Relationships: is a type of GO:0070566 Sources: RHEA:21360 Also known as: ATP:nicotinamide-nucleotide adenylyltransferase activity, NAD(+) diphosphorylase activity, NAD(+) pyrophosphorylase activity, NMN adenylyltransferase activity, NMNAT activity, nicotinamide adenine dinucleotide pyrophosphorylase activity, nicotinamide mononucleotide adenylyltransferase activity, ATP:NMN adenylyltransferase activity, NAD+ diphosphorylase activity, NAD+ pyrophosphorylase activity, adenosine triphosphate-nicotinamide mononucleotide transadenylase activity, diphosphopyridine nucleotide pyrophosphorylase activity Definition: Catalysis of the reaction: beta-nicotinamide D-ribonucleotide + ATP + H+ = diphosphate + NAD+.